{
  "gene_name": "HLA class I histocompatibility antigen, C alpha chain",
  "term_label": "antigen processing and presentation of endogenous peptide antigen via MHC class I via ER pathway, TAP-independent",
  "term_id": "GO:0002486",
  "gene_symbol": "HLA-C",
  "gene": "UniProtKB:P10321"
}